{
  "term_label": "action potential",
  "gene_symbol": "KCNG2",
  "term_id": "GO:0001508",
  "gene": "UniProtKB:Q9UJ96",
  "gene_name": "Potassium voltage-gated channel subfamily G member 2"
}